{
  "term_label": "Unknown molecular function",
  "gene": "UniProtKB:Q5TC04",
  "gene_symbol": "ATP1A1-AS1",
  "gene_name": "Putative uncharacterized protein ATP1A1-AS1",
  "term_id": "UNKNOWN:0001"
}